regulation of glycoprotein metabolic process [GO:1903018] (biological process) Definition: Any process that modulates the frequency, rate or extent of glycoprotein metabolic process. References: PMID:23544079 Sources: GOC:BHF, GOC:TermGenie, GOC:rl, GO_REF:0000058 Also known as: regulation of glycoprotein metabolism Note: human serum amyloid P component (SAP) P02743 inhibits viral neuraminidase, NA (exo-alpha-sialidase activity) and thus the metabolism of glycoproteins, demonstrated in Figure 4A PMID:23544079, (IDA), the negative regulation term would be applied to this protein Relationships: is a type of GO:0051246; regulates GO:0009100 Subtypes: regulation of glycoprotein biosynthetic process [GO:0010559], regulation of elastin catabolic process [GO:0060310], negative regulation of glycoprotein metabolic process [GO:1903019], positive regulation of glycoprotein metabolic process [GO:1903020]